{
  "gene": "UniProtKB:Q6BAA4",
  "gene_name": "Fc receptor-like B",
  "term_label": "immunoglobulin mediated immune response",
  "gene_symbol": "FCRLB",
  "term_id": "GO:0016064"
}